{
  "gene": "UniProtKB:Q8NFI4",
  "gene_name": "Putative protein FAM10A5",
  "term_id": "UNKNOWN:0002",
  "gene_symbol": "ST13P5",
  "term_label": "Unknown biological process"
}